{
  "gene_symbol": "STX10",
  "term_label": "endomembrane system",
  "gene_name": "Syntaxin-10",
  "term_id": "GO:0012505",
  "gene": "UniProtKB:O60499"
}